{
  "gene_symbol": "SAMD9",
  "term_label": "Unknown biological process",
  "gene": "UniProtKB:Q5K651",
  "term_id": "UNKNOWN:0002",
  "gene_name": "Sterile alpha motif domain-containing protein 9"
}